{
  "gene_symbol": "NFATC3",
  "term_label": "calcineurin-NFAT signaling cascade",
  "gene": "UniProtKB:Q12968",
  "term_id": "GO:0033173",
  "gene_name": "Nuclear factor of activated T-cells, cytoplasmic 3"
}